{
  "gene": "UniProtKB:Q9BTD1",
  "term_id": "UNKNOWN:0003",
  "gene_symbol": "SHANK2-AS3",
  "gene_name": "Putative uncharacterized protein SHANK2-AS3",
  "term_label": "Unknown cellular component"
}